{
  "term_id": "GO:0045892",
  "term_label": "negative regulation of DNA-templated transcription",
  "gene": "UniProtKB:Q8N5F7",
  "gene_symbol": "NKAP",
  "gene_name": "NF-kappa-B-activating protein"
}